interleukin-11 receptor binding [GO:0005142] (molecular function) Also known as: IL-11, interleukin-11 receptor ligand Definition: Binding to an interleukin-11 receptor. Relationships: is a type of cytokine receptor binding [GO:0005126]; is a type of growth factor receptor binding [GO:0070851] Sources: GOC:ai